regulation of peptide hormone processing [GO:0060568] (biological process) Subtypes: positive regulation of peptide hormone processing [GO:0060569], GO:0060570 Relationships: is a type of regulation of hormone metabolic process [GO:0032350]; is a type of regulation of amide metabolic process [GO:0034248]; is_a GO:0070613; regulates peptide hormone processing [GO:0016486] Definition: Any process that modulates the rate, frequency or extent of peptide hormone processing. Peptide hormone processing is the generation of a mature peptide hormone by posttranslational processing of a prohormone. Sources: GOC:dph, GOC:tb